{
  "gene_symbol": "TLK2",
  "term_id": "GO:0007059",
  "term_label": "chromosome segregation",
  "gene": "UniProtKB:Q86UE8",
  "gene_name": "Serine_threonine-protein kinase tousled-like 2"
}